{
  "term_id": "GO:0005634",
  "gene_symbol": "SS18L1",
  "term_label": "nucleus",
  "gene_name": "Calcium-responsive transactivator",
  "gene": "UniProtKB:O75177"
}